equatorial microtubule organizing center disassembly [GO:0031025] (biological process) References: PMID:15068790 Sources: GOC:mah Relationships: is_a GO:0022411; is_a microtubule organizing center organization [GO:0031023]; is a type of equatorial microtubule organization [GO:0031121] Also known as: equatorial microtubule organising center disassembly Definition: The process in which the equatorial microtubule organizing center is disassembled at the end of mitosis.